stress response to acid chemical [GO:0097532] (biological process) Subtypes: cellular stress response to acid chemical [GO:0097533] Relationships: is a type of GO:0001101; is a type of response to stress [GO:0006950] Also known as: response to acid stress, stress response to acid Definition: Any process that results in a change in state or activity of a cell or an organism (in terms of movement, secretion, enzyme production, gene expression, etc.) as a result of a disturbance in organismal or cellular homeostasis caused by the chemical structure of the anion portion of a dissociated acid (rather than the acid acting as a proton donor). The acid chemical may be in gaseous, liquid or solid form. References: PMID:10615049, PMID:19170886 Sources: GOC:BHF, GOC:aa, GOC:go_curators, GOC:rl, Wikipedia:Acid